{
  "gene": "UniProtKB:Q14469",
  "gene_symbol": "HES1",
  "term_label": "regulation of neurogenesis",
  "gene_name": "Transcription factor HES-1",
  "term_id": "GO:0050767"
}